{
  "term_label": "focal adhesion",
  "gene_symbol": "VASP",
  "term_id": "GO:0005925",
  "gene": "UniProtKB:P50552",
  "gene_name": "Vasodilator-stimulated phosphoprotein"
}